positive regulation of binding [GO:0051099] (biological process) Subtypes: positive regulation of protein binding [GO:0032092], GO:0035563, GO:0043388, positive regulation of GTP binding [GO:1904426], negative regulation of guanyl-nucleotide exchange factor activity [GO:1905098], GO:1905216 Also known as: up regulation of binding, up-regulation of binding, upregulation of binding, activation of binding, stimulation of binding Relationships: is a type of positive regulation of molecular function [GO:0044093]; is a type of regulation of binding [GO:0051098]; positively regulates binding [GO:0005488] Sources: GOC:ai Definition: Any process that activates or increases the rate or extent of binding, the selective interaction of a molecule with one or more specific sites on another molecule.